5-dehydro-2-deoxygluconokinase activity [GO:0047590] (molecular function) Relationships: is a type of kinase activity [GO:0016301]; is a type of phosphotransferase activity, alcohol group as acceptor [GO:0016773] Also known as: 5-keto-2-deoxyglucono kinase (phosphorylating), 5-keto-2-deoxygluconokinase activity, ATP:5-dehydro-2-deoxy-D-gluconate 6-phosphotransferase activity, DKH kinase activity Sources: EC:2.7.1.92, MetaCyc:5-DEHYDRO-2-DEOXYGLUCONOKINASE-RXN Definition: Catalysis of the reaction: ATP + 5-dehydro-2-deoxy-D-gluconate = ADP + 6-phospho-5-dehydro-2-deoxy-D-gluconate.